invasive growth in response to heat [GO:0036165] (biological process) Definition: The growth of colonies in filamentous chains of cells as a result of an increase in temperature. References: PMID:22365851 Sources: GOC:di Also known as: invasive growth in response to temperature stimulus, invasive growth in response to elevated temperature, invasive growth in response to high temperature Relationships: is a type of GO:0036168; is a type of invasive filamentous growth [GO:0036267]